{
  "gene": "UniProtKB:Q96G28",
  "term_label": "Unknown biological process",
  "gene_name": "Cilia- and flagella-associated protein 36",
  "term_id": "UNKNOWN:0002",
  "gene_symbol": "CFAP36"
}